{
  "gene_name": "Transcription initiation factor TFIID subunit 3",
  "term_id": "GO:0002039",
  "gene_symbol": "TAF3",
  "gene": "UniProtKB:Q5VWG9",
  "term_label": "p53 binding"
}